{
  "term_id": "GO:0038163",
  "gene_name": "Thrombopoietin receptor",
  "gene_symbol": "MPL",
  "gene": "UniProtKB:P40238",
  "term_label": "thrombopoietin-mediated signaling pathway"
}